response to bleomycin [GO:1904975] (biological process) Relationships: is a type of response to nitrogen compound [GO:1901698]; is a type of response to oxygen-containing compound [GO:1901700] Definition: Any process that results in a change in state or activity of a cell or an organism (in terms of movement, secretion, enzyme production, gene expression, etc.) as a result of a bleomycin stimulus. References: PMID:11553781 Sources: GOC:TermGenie, GO_REF:0000071 Subtypes: cellular response to bleomycin [GO:1904976]